{
  "gene": "UniProtKB:P0DW12",
  "term_id": "GO:0016251",
  "gene_symbol": "TAF11L7",
  "term_label": "RNA polymerase II general transcription initiation factor activity",
  "gene_name": "TATA-box-binding protein-associated factor 11-like protein 7"
}